trans-synaptic signaling by carbon monoxide, modulating synaptic transmission [GO:0099556] (biological process) Definition: Cell-cell signaling between presynapse and postsynapse, via the release and reception of carbon monoxide molecules, that modulates the synaptic transmission properties of the synapse. Sources: GOC:dos Note: Note that this term was created for the SynGO project, and will be obsoleted when the SynGO annotations are made in Noctua. Relationships: is a type of trans-synaptic signaling by carbon monoxide [GO:0099549]; is a type of trans-synaptic signaling by soluble gas, modulating synaptic transmission [GO:0099554]